protein-arginine C-methyltransferase activity [GO:0035244] (MF) Definition: Catalysis of the transfer of a methyl group to the carbon atom of an arginine residue in a protein. This modification has been detected in anaerobic bacteria. Also known as: peptidyl arginine C-methyltransferase activity, peptidyl-arginine C-methylase activity, peptidyl-arginine C-methyltransferase activity, protein-arginine C-methylase activity Relationships: is a type of GO:0008169; is a type of protein methyltransferase activity [GO:0008276]; is a type of S-adenosylmethionine-dependent methyltransferase activity [GO:0008757] References: PMID:29743535, PMID:33162960 Sources: GOC:bf, RHEA:66028